{
  "term_label": "vesicle cytoskeletal trafficking",
  "term_id": "GO:0099518",
  "gene_name": "Coiled-coil domain-containing protein 186",
  "gene_symbol": "CCDC186",
  "gene": "UniProtKB:Q7Z3E2"
}